{
  "gene": "UniProtKB:Q8N0S6",
  "gene_name": "Centromere protein L",
  "gene_symbol": "CENPL",
  "term_label": "Unknown cellular component",
  "term_id": "UNKNOWN:0003"
}